{
  "gene_symbol": "CAPRIN1",
  "gene": "UniProtKB:Q14444",
  "term_id": "UNKNOWN:0002",
  "term_label": "Unknown biological process",
  "gene_name": "Caprin-1"
}